{
  "term_id": "GO:0007423",
  "term_label": "sensory organ development",
  "gene": "UniProtKB:P50553",
  "gene_name": "Achaete-scute homolog 1",
  "gene_symbol": "ASCL1"
}